{
  "gene_symbol": "ATL1",
  "gene": "UniProtKB:Q8WXF7",
  "term_label": "protein homooligomerization",
  "term_id": "GO:0051260",
  "gene_name": "Atlastin-1"
}